{
  "term_label": "endoplasmic reticulum membrane",
  "gene_symbol": "TMEM41B",
  "term_id": "GO:0005789",
  "gene_name": "Transmembrane protein 41B",
  "gene": "UniProtKB:Q5BJD5"
}